{
  "term_id": "GO:1904263",
  "term_label": "positive regulation of TORC1 signaling",
  "gene_symbol": "RRAGB",
  "gene": "UniProtKB:Q5VZM2",
  "gene_name": "Ras-related GTP-binding protein B"
}